{
  "gene": "UniProtKB:P31943",
  "term_id": "GO:1990904",
  "gene_symbol": "HNRNPH1",
  "gene_name": "Heterogeneous nuclear ribonucleoprotein H",
  "term_label": "ribonucleoprotein complex"
}